{
  "gene_symbol": "ENKUR",
  "gene_name": "Enkurin",
  "term_id": "GO:0001669",
  "term_label": "acrosomal vesicle",
  "gene": "UniProtKB:Q8TC29"
}